cardiac epithelial to mesenchymal transition [GO:0060317] (biological process) Also known as: heart epithelial to mesenchymal transition Subtypes: epithelial to mesenchymal transition involved in endocardial cushion formation [GO:0003198], epithelial to mesenchymal transition involved in coronary vasculature morphogenesis [GO:0003201], GO:0060940, GO:0090500 References: PMID:16314491, PMID:1996351 Sources: GOC:BHF, GOC:dph Regulation: regulated by regulation of cardiac epithelial to mesenchymal transition [GO:0062042]; positively regulated by positive regulation of cardiac epithelial to mesenchymal transition [GO:0062043]; RO_0002212 by negative regulation of cardiac epithelial to mesenchymal transition [GO:0062044] Relationships: is a type of epithelial to mesenchymal transition [GO:0001837]; BFO_0000050 heart morphogenesis [GO:0003007] Definition: A transition where a cardiac epithelial cell loses apical/basolateral polarity, severs intercellular adhesive junctions, degrades basement membrane components and becomes a migratory mesenchymal cell.